{
  "term_id": "GO:0001837",
  "term_label": "epithelial to mesenchymal transition",
  "gene_name": "Transforming growth factor beta receptor type 3",
  "gene": "UniProtKB:Q03167",
  "gene_symbol": "TGFBR3"
}